{
  "gene": "UniProtKB:A0A0G2JN53",
  "term_label": "Unknown molecular function",
  "gene_symbol": "A0A0G2JN53",
  "term_id": "UNKNOWN:0001",
  "gene_name": "IQ motif and SEC7 domain-containing protein 3"
}